{
  "term_label": "endoplasmic reticulum",
  "term_id": "GO:0005783",
  "gene_symbol": "CYB5R4",
  "gene_name": "Cytochrome b5 reductase 4",
  "gene": "UniProtKB:Q7L1T6"
}